extrinsic apoptotic signaling pathway in absence of ligand [GO:0097192] (biological process) Note: For dependence receptors, absence of a ligand or withdrawal of a ligand from a receptor acts as a signal. An example of 'extrinsic apoptotic signaling pathway in absence of ligand' is withdrawal of a growth factor such as NGF, even if traditionally apoptosis induced via growth factor withdrawal has been classified as an instance of intrinsic apoptosis. See an example in PMID:19767770. Ligands whose withdrawal or absence induce apoptosis should be annotated to GO:2001239 'regulation of extrinsic apoptotic signaling pathway in absence of ligand', rather than to the pathway term itself. Examples of gene products that may be annotated to GO:0097192 'extrinsic apoptotic signaling pathway in absence of ligand' include dependence receptors such as DCC or UNC5B, which relay lethal signals in the absence of their ligand (netrin-1). In the case of DCC and UNC5B, the signaling proceeds through the assembly of a DRAL- and TUCAN- (or NLRP1-) containing caspase-9-activating complex or by the dephosphorylation-mediated activation of death-associated protein kinase 1 (DAPK1) by UNC5B-bound protein phosphatase 2A (PP2A), respectively. DAPK1 can mediate the direct activation of executioner caspases or favor MOMP (reviewed in PMID:21760595). Also see PMID:21172653 (annotations to UNC5B and PR65beta, UniProt symbols O08722, PPP2R1B and P30154). Relationships: is a type of signal transduction in absence of ligand [GO:0038034]; is_a extrinsic apoptotic signaling pathway [GO:0097191] Also known as: extrinsic apoptotic signalling pathway in absence of ligand, extrinsic apoptosis in absence of ligand, dependence receptor signaling pathway Definition: The series of molecular signals in which a signal is conveyed from the cell surface to trigger the apoptotic death of a cell. The pathway starts with withdrawal of a ligand from a cell surface receptor, and ends when the execution phase of apoptosis is triggered. Regulation: regulated by regulation of extrinsic apoptotic signaling pathway in absence of ligand [GO:2001239]; negatively regulated by GO:2001240; positively regulated by positive regulation of extrinsic apoptotic signaling pathway in absence of ligand [GO:2001241] References: PMID:15044679, PMID:20816705 Sources: GOC:mtg_apoptosis